{
  "gene": "UniProtKB:Q15283",
  "gene_symbol": "RASA2",
  "term_label": "GTPase activator activity",
  "gene_name": "Ras GTPase-activating protein 2",
  "term_id": "GO:0005096"
}